IgD B cell receptor complex [GO:0071740] (cellular component) Relationships: is a type of GO:0019815; is_a IgD immunoglobulin complex [GO:0071738] Note: Note that an IgD immunoglobulin complex has the function of antigen binding if a suitable antigen is available. References: PMID:11282392 Sources: GOC:add, ISBN:0781765196 Definition: An IgD immunoglobulin complex that is present in the plasma membrane of B cells and is composed of two identical immunoglobulin heavy chains of the IgD isotype and two identical immunoglobulin light chains and a signaling subunit, a heterodimer of the Ig-alpha and Ig-beta proteins. Also known as: membrane-bound IgD, surface IgD